{
  "term_id": "GO:0005737",
  "term_label": "cytoplasm",
  "gene_name": "GRB2-related adapter protein",
  "gene": "UniProtKB:Q13588",
  "gene_symbol": "GRAP"
}